{
  "term_label": "Unknown molecular function",
  "term_id": "UNKNOWN:0001",
  "gene": "UniProtKB:Q9BZJ0",
  "gene_symbol": "CRNKL1",
  "gene_name": "Crooked neck-like protein 1"
}